{
  "term_label": "plasma membrane",
  "gene_name": "Olfactory receptor 4A47",
  "term_id": "GO:0005886",
  "gene_symbol": "OR4A47",
  "gene": "UniProtKB:Q6IF82"
}